imaginal disc-derived wing hair site selection [GO:0035320] (biological process) Also known as: wing hair site selection, prehair localization Relationships: is a type of establishment of proximal/distal cell polarity [GO:0022606]; is part of establishment of imaginal disc-derived wing hair orientation [GO:0001737] Definition: Determination of the site in the cell of an imaginal disc-derived wing at which a prehair initiates outgrowth. Restriction of prehair initiation to the distalmost part of a cell is essential to ensure that each wing epithelial cell produces one adult hair that points distally. References: PMID:8947551 Sources: GOC:mtg_transport, ISBN:0815340729